lysosome [GO:0005764] (cellular component) Relationships: is a type of lytic vacuole [GO:0000323] Sources: GOC:mah, ISBN:0198506732 Definition: A small lytic vacuole that has cell cycle-independent morphology found in most animal cells and that contains a variety of hydrolases, most of which have their maximal activities in the pH range 5-6. The contained enzymes display latency if properly isolated. About 40 different lysosomal hydrolases are known and lysosomes have a great variety of morphologies and functions. Subtypes: GO:0005766, secondary lysosome [GO:0005767], endolysosome [GO:0036019], mast cell granule [GO:0042629], megasome [GO:0043246], cytolytic granule [GO:0044194]